glycerophosphocholine phosphodiesterase activity [GO:0047389] (molecular function) Relationships: is a type of phosphoric diester hydrolase activity [GO:0008081] Also known as: glycerolphosphorylcholine phosphodiesterase activity, glycerophosphinicocholine diesterase activity, glycerophosphohydrolase activity, glycerylphosphorylcholinediesterase activity, sn-glycero-3-phosphocholine glycerophosphohydrolase activity, sn-glycero-3-phosphorylcholine diesterase activity Definition: Catalysis of the reaction: H2O + L-1-glycero-3-phosphocholine = glycerol-3-phosphate + choline. Sources: EC:3.1.4.2, MetaCyc:3.1.4.2-RXN